{
  "gene": "UniProtKB:O43159",
  "term_label": "chromatin silencing complex",
  "gene_name": "Ribosomal RNA-processing protein 8",
  "gene_symbol": "RRP8",
  "term_id": "GO:0005677"
}